{
  "gene_symbol": "ANAPC4",
  "gene": "UniProtKB:Q9UJX5",
  "gene_name": "Anaphase-promoting complex subunit 4",
  "term_label": "protein K11-linked ubiquitination",
  "term_id": "GO:0070979"
}